{
  "gene_symbol": "OR2M3",
  "term_id": "GO:0005886",
  "gene_name": "Olfactory receptor 2M3",
  "gene": "UniProtKB:Q8NG83",
  "term_label": "plasma membrane"
}